{
  "gene": "UniProtKB:Q8NGZ5",
  "gene_symbol": "OR2G2",
  "term_id": "GO:0004984",
  "term_label": "olfactory receptor activity",
  "gene_name": "Olfactory receptor 2G2"
}